{
  "term_id": "GO:0007193",
  "gene_symbol": "GPR176",
  "term_label": "adenylate cyclase-inhibiting G protein-coupled receptor signaling pathway",
  "gene": "UniProtKB:Q14439",
  "gene_name": "G-protein coupled receptor 176"
}